{
  "term_id": "GO:0042800",
  "term_label": "histone H3K4 methyltransferase activity",
  "gene": "UniProtKB:Q9UMN6",
  "gene_name": "Histone-lysine N-methyltransferase 2B",
  "gene_symbol": "KMT2B"
}